bone resorption [GO:0045453] (biological process) References: PMID:10968780 Sources: GOC:mah Relationships: is a type of tissue homeostasis [GO:0001894]; BFO_0000050 bone remodeling [GO:0046849] Definition: The process in which specialized cells known as osteoclasts degrade the organic and inorganic portions of bone, and endocytose and transport the degradation products. Regulation: regulated by regulation of bone resorption [GO:0045124]; negatively regulated by negative regulation of bone resorption [GO:0045779]; positively regulated by positive regulation of bone resorption [GO:0045780]